{
  "gene": "UniProtKB:Q5EG05",
  "gene_name": "Caspase recruitment domain-containing protein 16",
  "gene_symbol": "CARD16",
  "term_label": "Unknown cellular component",
  "term_id": "UNKNOWN:0003"
}